smooth muscle cell proliferation [GO:0048659] (biological process) Also known as: SMC proliferation Regulation: regulated by regulation of smooth muscle cell proliferation [GO:0048660]; positively regulated by positive regulation of smooth muscle cell proliferation [GO:0048661]; negatively regulated by negative regulation of smooth muscle cell proliferation [GO:0048662] Subtypes: GO:1990874 Relationships: is a type of muscle cell proliferation [GO:0033002] References: PMID:1840698 Sources: CL:0000192, GOC:ebc Definition: The multiplication or reproduction of smooth muscle cells, resulting in the expansion of a cell population.